{
  "term_label": "lipid metabolic process",
  "gene": "UniProtKB:Q6ZPD8",
  "gene_name": "Diacylglycerol O-acyltransferase 2-like protein 6",
  "term_id": "GO:0006629",
  "gene_symbol": "DGAT2L6"
}